{
  "term_id": "GO:0038084",
  "gene_name": "Vascular endothelial growth factor C",
  "term_label": "vascular endothelial growth factor signaling pathway",
  "gene_symbol": "VEGFC",
  "gene": "UniProtKB:P49767"
}